{
  "gene_symbol": "ZNF562",
  "gene": "UniProtKB:Q6V9R5",
  "term_label": "DNA-binding transcription factor activity, RNA polymerase II-specific",
  "term_id": "GO:0000981",
  "gene_name": "Zinc finger protein 562"
}